positive regulation of inhibitory synapse assembly [GO:1905704] (biological process) Relationships: is a type of positive regulation of synapse assembly [GO:0051965]; is a type of GO:1905702; positively regulates inhibitory synapse assembly [GO:1904862] Also known as: positive regulation of inhibitory synapse formation, up regulation of inhibitory synapse assembly, up regulation of inhibitory synapse formation, up-regulation of inhibitory synapse assembly, up-regulation of inhibitory synapse formation, upregulation of inhibitory synapse assembly, upregulation of inhibitory synapse formation, activation of inhibitory synapse assembly, activation of inhibitory synapse formation Definition: Any process that activates or increases the frequency, rate or extent of inhibitory synapse assembly. References: PMID:27779093 Sources: GOC:TermGenie, GO_REF:0000058